{
  "term_label": "nucleolus",
  "gene_name": "Terminal nucleotidyltransferase 4A",
  "term_id": "GO:0005730",
  "gene": "UniProtKB:Q5XG87",
  "gene_symbol": "TENT4A"
}